membrane protein ectodomain proteolysis [GO:0006509] (biological process) Regulation: RO_0002211 by regulation of membrane protein ectodomain proteolysis [GO:0051043]; positively regulated by positive regulation of membrane protein ectodomain proteolysis [GO:0051044]; negatively regulated by negative regulation of membrane protein ectodomain proteolysis [GO:0051045] Definition: The proteolytic cleavage of transmembrane proteins and release of their ectodomain (extracellular domain). Also known as: ectoderm shedding, ectodomain cleavage, membrane protein solubilization, receptor shedding References: PMID:24227200 Sources: GOC:jl Relationships: is a type of membrane protein proteolysis [GO:0033619] Subtypes: constitutive protein ectodomain proteolysis [GO:0051089]